cell septum assembly [GO:0090529] (biological process) Sources: GOC:mtg_cell_cycle Regulation: regulated by regulation of cell septum assembly [GO:1901891]; negatively regulated by negative regulation of cell septum assembly [GO:1901892]; positively regulated by GO:1901893 Subtypes: division septum assembly [GO:0000917] Relationships: is a type of GO:0022607; is a type of cytokinetic process [GO:0032506] Definition: The assembly and arrangement of a cellular component that is composed of peptidoglycan and often chitin in addition to other materials and usually forms perpendicular to the long axis of a cell or hypha. It grows centripetally from the cell wall to the center of the cell and often functions in the compartmentalization of a cell into two daughter cells. Also known as: cell septum assembly involved in cell cycle cytokinesis